{
  "term_label": "cellular response to nitrogen starvation",
  "term_id": "GO:0006995",
  "gene_symbol": "GABARAPL2",
  "gene": "UniProtKB:P60520",
  "gene_name": "Gamma-aminobutyric acid receptor-associated protein-like 2"
}